ventricular cardiac muscle tissue development [GO:0003229] (biological process) Sources: GOC:mtg_heart Subtypes: His-Purkinje system development [GO:0003164], Purkinje myocyte development [GO:0003165], bundle of His development [GO:0003166] Also known as: ventricular myocardium development Relationships: is a type of cardiac muscle tissue development [GO:0048738] Definition: The process whose specific outcome is the progression of ventricular cardiac muscle over time, from its formation to the mature structure.